{
  "term_id": "GO:0006909",
  "gene_name": "Neutrophil elastase",
  "gene_symbol": "ELANE",
  "term_label": "phagocytosis",
  "gene": "UniProtKB:P08246"
}